{
  "gene_symbol": "PAM",
  "gene": "UniProtKB:P19021",
  "term_id": "UNKNOWN:0002",
  "gene_name": "Peptidyl-glycine alpha-amidating monooxygenase",
  "term_label": "Unknown biological process"
}